gastric mucosal blood circulation [GO:1990768] (BP) Also known as: stomach mucosal blood circulation References: PMID:10807413 Regulation: regulated by regulation of gastric mucosal blood circulation [GO:1904344]; negatively regulated by negative regulation of gastric mucosal blood circulation [GO:1904345]; RO_0002213 by positive regulation of gastric mucosal blood circulation [GO:1904346] Definition: The flow of blood through the gastric mucosa of an animal, enabling the transport of nutrients and the removal of waste products. Relationships: is a type of GO:0008015